distal dendrite [GO:0150002] (cellular component) Definition: The dendrite of the dendritic tree that is farthest away from the neuronal cell body (the soma). Relationships: is a type of dendrite [GO:0030425] Subtypes: apical distal dendrite [GO:0150014], basal distal dendrite [GO:0150016] References: PMID:20629984 Sources: GOC:aruk, GOC:bc